{
  "gene": "UniProtKB:Q9UMR3",
  "term_label": "regulation of transcription by RNA polymerase II",
  "term_id": "GO:0006357",
  "gene_symbol": "TBX20",
  "gene_name": "T-box transcription factor TBX20"
}